{
  "gene_name": "Immunoglobulin heavy constant alpha 1",
  "term_label": "immunoglobulin complex, circulating",
  "gene": "UniProtKB:P01876",
  "term_id": "GO:0042571",
  "gene_symbol": "IGHA1"
}